{
  "gene_symbol": "OR5M1",
  "gene": "UniProtKB:Q8NGP8",
  "term_id": "UNKNOWN:0003",
  "term_label": "Unknown cellular component",
  "gene_name": "Olfactory receptor 5M1"
}